{
  "term_label": "microtubule severing",
  "gene_symbol": "FIGN",
  "gene_name": "Fidgetin",
  "term_id": "GO:0051013",
  "gene": "UniProtKB:Q5HY92"
}